{
  "term_id": "UNKNOWN:0003",
  "gene_name": "Tetratricopeptide repeat protein 23-like",
  "gene": "UniProtKB:Q6PF05",
  "gene_symbol": "TTC23L",
  "term_label": "Unknown cellular component"
}